{
  "gene_symbol": "SRRM1",
  "gene_name": "Serine_arginine repetitive matrix protein 1",
  "term_id": "GO:0005681",
  "term_label": "spliceosomal complex",
  "gene": "UniProtKB:Q8IYB3"
}